{
  "gene_symbol": "AGTR2",
  "term_id": "GO:0042311",
  "gene": "UniProtKB:P50052",
  "term_label": "vasodilation",
  "gene_name": "Type-2 angiotensin II receptor"
}